{
  "term_label": "Unknown biological process",
  "gene_name": "Nucleoporin NUP42",
  "gene": "UniProtKB:O15504",
  "term_id": "UNKNOWN:0002",
  "gene_symbol": "NUP42"
}